{
  "term_label": "P granule",
  "gene_symbol": "HELZ2",
  "term_id": "GO:0043186",
  "gene_name": "Helicase with zinc finger domain 2",
  "gene": "UniProtKB:Q9BYK8"
}